ferric iron binding [GO:0008199] (molecular function) Sources: GOC:ai Relationships: is a type of iron ion binding [GO:0005506] Definition: Binding to a ferric iron ion, Fe(III).